{
  "gene_name": "Zinc finger protein 12",
  "gene_symbol": "ZNF12",
  "gene": "UniProtKB:P17014",
  "term_id": "GO:0006357",
  "term_label": "regulation of transcription by RNA polymerase II"
}